{
  "gene_symbol": "EXOSC2",
  "term_label": "nuclear exosome (RNase complex)",
  "gene_name": "Exosome complex component RRP4",
  "gene": "UniProtKB:Q13868",
  "term_id": "GO:0000176"
}